protein O-linked glycosylation via mannose [GO:0035269] (BP) References: PMID:35536928 Relationships: is_a protein O-linked glycosylation [GO:0006493] Definition: A glycoprotein biosynthetic process starting with the covalent linkage of a mannose via an alpha-glycosidic bond to the oxygen atom of a serine or threonine side chain in a protein, which can be further elongated with the sequential addition of sugar units resulting in the formation of a protein O-linked glycan. Subtypes: GO:0140265 Also known as: protein amino acid O-linked mannosylation, protein O-linked mannosylation